{
  "term_label": "ciliary transition zone",
  "gene_name": "Meckelin",
  "gene_symbol": "TMEM67",
  "gene": "UniProtKB:Q5HYA8",
  "term_id": "GO:0035869"
}